{
  "gene": "UniProtKB:P14316",
  "term_id": "GO:0006357",
  "term_label": "regulation of transcription by RNA polymerase II",
  "gene_symbol": "IRF2",
  "gene_name": "Interferon regulatory factor 2"
}